transforming growth factor beta2 production [GO:0032906] (BP) Regulation: regulated by regulation of transforming growth factor beta2 production [GO:0032909]; negatively regulated by negative regulation of transforming growth factor beta2 production [GO:0032912]; positively regulated by positive regulation of transforming growth factor beta2 production [GO:0032915] Definition: The appearance of transforming growth factor-beta2 due to biosynthesis or secretion following a cellular stimulus, resulting in an increase in its intracellular or extracellular levels. Sources: GOC:mah Also known as: TGF-B2 production, TGFB2 production, transforming growth factor-beta2 production Relationships: is a type of transforming growth factor beta production [GO:0071604]